dorsal appendage formation [GO:0046843] (biological process) Definition: Establishment of the dorsal filaments, elaborate specializations of the chorion that protrude from the anterior end of the egg and facilitate embryonic respiration. Sources: ISBN:0879694238 Relationships: is a type of developmental process involved in reproduction [GO:0003006]; is a type of anatomical structure formation involved in morphogenesis [GO:0048646]; is part of GO:0007306